response to host immune response [GO:0052572] (biological process) Sources: GOC:mtg_pamgo_17jul06 Subtypes: symbiont-mediated evasion of host immune response [GO:0042783] Also known as: response to immune response of other organism involved in symbiotic interaction Definition: Any process that results in a change in state or activity of a cell or an organism (in terms of movement, secretion, enzyme production, gene expression, etc.) as a result of detecting the immune response of the host organism. The host is defined as the larger of the organisms involved in a symbiotic interaction. Relationships: is a type of symbiont-mediated response to host defenses [GO:0052200]